{
  "gene": "UniProtKB:Q9NP50",
  "term_label": "Sin3-type complex",
  "gene_symbol": "SINHCAF",
  "gene_name": "SIN3-HDAC complex-associated factor",
  "term_id": "GO:0070822"
}